{
  "term_id": "GO:0003712",
  "gene_name": "Akirin-1",
  "gene": "UniProtKB:Q9H9L7",
  "gene_symbol": "AKIRIN1",
  "term_label": "transcription coregulator activity"
}